{
  "gene_symbol": "FSCN2",
  "gene": "UniProtKB:O14926",
  "term_id": "GO:0015629",
  "term_label": "actin cytoskeleton",
  "gene_name": "Fascin-2"
}